{
  "gene_symbol": "OR6S1",
  "gene": "UniProtKB:Q8NH40",
  "term_label": "Unknown biological process",
  "gene_name": "Olfactory receptor 6S1",
  "term_id": "UNKNOWN:0002"
}